spinal trigeminal nucleus development [GO:0021741] (biological process) Relationships: is a type of GO:0021730 Sources: GOC:cls, GOC:curators, GOC:dgh, GOC:dph, GOC:jid Definition: The process whose specific outcome is the progression of the spinal trigeminal nucleus over time, from its formation to the mature structure.